negative regulation of CD8-positive, alpha-beta T cell activation [GO:2001186] (biological process) Definition: Any process that stops, prevents or reduces the frequency, rate or extent of CD8-positive, alpha-beta T cell activation. Subtypes: GO:0043377, negative regulation of CD8-positive, alpha-beta T cell proliferation [GO:2000565] Sources: GOC:obol Relationships: is_a GO:0046636; is a type of regulation of CD8-positive, alpha-beta T cell activation [GO:2001185]; negatively regulates GO:0036037